{
  "gene_symbol": "CTXND2",
  "gene": "UniProtKB:A0A1B0GV90",
  "gene_name": "Cortexin domain containing 2",
  "term_label": "Unknown cellular component",
  "term_id": "UNKNOWN:0003"
}